{
  "term_id": "GO:0006955",
  "gene_symbol": "CLEC10A",
  "term_label": "immune response",
  "gene": "UniProtKB:Q8IUN9",
  "gene_name": "C-type lectin domain family 10 member A"
}